{
  "term_label": "Unknown cellular component",
  "gene_name": "Pre-mRNA-splicing factor ATP-dependent RNA helicase DHX16",
  "term_id": "UNKNOWN:0003",
  "gene": "UniProtKB:O60231",
  "gene_symbol": "DHX16"
}